{
  "term_id": "GO:0007019",
  "gene_symbol": "KATNB1",
  "gene": "UniProtKB:Q9BVA0",
  "term_label": "microtubule depolymerization",
  "gene_name": "Katanin p80 WD40 repeat-containing subunit B1"
}